{
  "term_id": "UNKNOWN:0001",
  "gene": "UniProtKB:O15117",
  "gene_name": "FYN-binding protein 1",
  "term_label": "Unknown molecular function",
  "gene_symbol": "FYB1"
}